{
  "term_label": "mRNA binding",
  "gene_name": "Protein Smaug homolog 2",
  "gene_symbol": "SAMD4B",
  "gene": "UniProtKB:Q5PRF9",
  "term_id": "GO:0003729"
}